{
  "term_label": "calcium-dependent phospholipid binding",
  "gene_name": "Annexin A10",
  "term_id": "GO:0005544",
  "gene_symbol": "ANXA10",
  "gene": "UniProtKB:Q9UJ72"
}